{
  "gene_name": "Septin-2",
  "term_id": "GO:0060271",
  "term_label": "cilium assembly",
  "gene": "UniProtKB:Q15019",
  "gene_symbol": "SEPTIN2"
}